{
  "term_label": "organic anion transport",
  "gene_symbol": "SLC22A10",
  "gene_name": "Solute carrier family 22 member 10",
  "term_id": "GO:0015711",
  "gene": "UniProtKB:Q63ZE4"
}